response to DDT [GO:0046680] (BP) Definition: Any process that results in a change in state or activity of a cell or an organism (in terms of movement, secretion, enzyme production, gene expression, etc.) as a result of a DDT stimulus. DDT, dichlorodiphenyltrichloroethane, is a chlorinated hydrocarbon pesticide moderately toxic to humans and other animals. Sources: ISBN:0721662544 Also known as: DDT resistance, DDT susceptibility/resistance Relationships: is a type of response to insecticide [GO:0017085]